{
  "gene_name": "Lethal(3)malignant brain tumor-like protein 3",
  "gene_symbol": "L3MBTL3",
  "term_id": "GO:0003682",
  "gene": "UniProtKB:Q96JM7",
  "term_label": "chromatin binding"
}